{
  "gene_name": "Signal transducer and activator of transcription 6",
  "term_id": "GO:0043434",
  "gene_symbol": "STAT6",
  "gene": "UniProtKB:P42226",
  "term_label": "response to peptide hormone"
}